Gemini of Cajal bodies [GO:0097504] (cellular component) Relationships: is a type of nuclear body [GO:0016604] Also known as: Gemini of coiled bodies, Gems Definition: Nuclear bodies frequently found near or associated with Cajal bodies (also called coiled bodies or CBs). Gemini of coiled bodies, or 'gems', are similar in size and shape to CBs, and often indistinguishable under the microscope. Unlike CBs, gems do not contain small nuclear ribonucleoproteins (snRNPs); they contain a protein called survivor of motor neurons (SMN) whose function relates to snRNP biogenesis. Gems are believed to assist CBs in snRNP biogenesis, and to play a role in the etiology of spinal muscular atrophy (SMA). References: PMID:11031238, PMID:9683623 Sources: GOC:pr, Wikipedia:Cell_nucleus#Cajal_bodies_and_gems